cardiac vascular smooth muscle cell development [GO:0060948] (biological process) Subtypes: epicardium-derived cardiac vascular smooth muscle cell development [GO:0060984] Relationships: is a type of cardiac cell development [GO:0055006]; is a type of vascular associated smooth muscle cell development [GO:0097084]; is part of GO:0060947 Definition: The process whose specific outcome is the progression of a cardiac vascular smooth muscle cell over time, from its formation to the mature state. Also known as: heart vascular smooth muscle cell development Sources: GOC:mtg_heart